{
  "term_id": "GO:0005737",
  "gene_symbol": "TIRAP",
  "term_label": "cytoplasm",
  "gene_name": "Toll_interleukin-1 receptor domain-containing adapter protein",
  "gene": "UniProtKB:P58753"
}